{
  "gene": "UniProtKB:Q9UH17",
  "term_id": "GO:0000932",
  "gene_symbol": "APOBEC3B",
  "gene_name": "DNA dC-dU-editing enzyme APOBEC-3B",
  "term_label": "P-body"
}